cytochrome bo3 ubiquinol oxidase activity [GO:0009486] (molecular function) Definition: Catalysis of the reaction: 2 ubiquinol + O2 + 4 H+ = 2 ubiquinone + 2 H2O + 4 H+ [periplasmic space]. Relationships: is a type of GO:0009055; is a type of GO:0015453; is a type of oxidoreductase activity, acting on a heme group of donors [GO:0016675] Sources: RHEA:30251 Also known as: cytochrome bo oxidase, cytochrome bo(3) oxidase, cytochrome o ubiquinol oxidase activity